{
  "term_label": "BMP signaling pathway",
  "gene_name": "Repulsive guidance molecule A",
  "term_id": "GO:0030509",
  "gene": "UniProtKB:Q96B86",
  "gene_symbol": "RGMA"
}